symbiont-mediated perturbation of host heat acclimation [GO:0033638] (biological process) Also known as: modulation by symbiont of host heat acclimation, modulation by symbiont of host response to heat, response to heat shock Relationships: is a type of symbiont-mediated perturbation of host response to abiotic stimulus [GO:0033635] References: PMID:17425405, PMID:35350854 Sources: GOC:pamgo_curators Definition: A process in which a symbiont alters or subverts the response of its host to heat acclimation. The host is defined as the larger of the organisms involved in a symbiotic interaction.